{
  "term_label": "aggresome",
  "gene_name": "E3 ubiquitin-protein ligase TRIM37",
  "gene_symbol": "TRIM37",
  "term_id": "GO:0016235",
  "gene": "UniProtKB:O94972"
}